{
  "gene_symbol": "ZFYVE21",
  "term_label": "Unknown molecular function",
  "gene": "UniProtKB:Q9BQ24",
  "term_id": "UNKNOWN:0001",
  "gene_name": "Zinc finger FYVE domain-containing protein 21"
}